{
  "term_label": "Unknown molecular function",
  "gene": "UniProtKB:Q2VPJ9",
  "gene_name": "Leucine-rich repeat-containing protein 75B",
  "gene_symbol": "LRRC75B",
  "term_id": "UNKNOWN:0001"
}